regulation of nitrogen cycle metabolic process [GO:1903314] (biological process) Sources: GOC:TermGenie, GOC:vw, GO_REF:0000058 Definition: Any process that modulates the frequency, rate or extent of nitrogen cycle metabolic process. Subtypes: GO:0034254, regulation of nitrate assimilation [GO:0090352], GO:1903315, positive regulation of nitrogen cycle metabolic process [GO:1903316] Relationships: is a type of GO:0019222; regulates nitrogen cycle metabolic process [GO:0071941]